{
  "term_label": "nucleus",
  "term_id": "GO:0005634",
  "gene": "UniProtKB:B1ANY3",
  "gene_name": "Putative protein FAM220BP",
  "gene_symbol": "FAM220BP"
}